{
  "term_label": "protein localization to plasma membrane",
  "gene_symbol": "C2CD5",
  "gene_name": "C2 domain-containing protein 5",
  "term_id": "GO:0072659",
  "gene": "UniProtKB:Q86YS7"
}